pseudouridylate synthase activity [GO:0004730] (molecular function) Definition: Catalysis of the reaction: D-ribose 5-phosphate + uracil = H2O + pseudouridine 5'-phosphate. Relationships: is a type of GO:0016836; is part of pseudouridine synthesis [GO:0001522] Sources: EC:4.2.1.70, RHEA:18337 Note: Note that this term should not be confused with 'pseudouridine synthase activity ; GO:0009982', which refers to the intramolecular isomerization of uridine to pseudouridine. Also known as: pseudouridine monophosphate synthase activity, pseudouridine-5'-phosphate glycosidase activity, 5-ribosyluracil 5-phosphate synthetase activity, pseudouridine monophosphate synthetase activity, pseudouridylate synthetase activity, pseudouridylic acid synthetase activity, psiUMP synthetase activity, uracil hydro-lyase (adding D-ribose 5-phosphate), uracil hydro-lyase (adding D-ribose 5-phosphate; pseudouridine-5'-phosphate-forming), uracil hydrolyase activity